{
  "term_id": "GO:0000398",
  "gene_name": "BUD13 homolog",
  "gene_symbol": "BUD13",
  "term_label": "mRNA splicing, via spliceosome",
  "gene": "UniProtKB:Q9BRD0"
}